nuclear pre-replicative complex [GO:0005656] (cellular component) Definition: A protein-DNA complex assembled at eukaryotic DNA replication origins during late mitosis and G1, allowing the origin to become competent, or 'licensed', for replication. The complex normally includes the origin recognition complex (ORC), Cdc6, Cdt1 and the MiniChromosome Maintenance (Mcm2-7) proteins. References: PMID:15222894 Also known as: pre-replicative complex, eukaryotic pre-replicative complex, pre-RC Relationships: is a type of pre-replicative complex [GO:0036387]; is a type of nuclear protein-containing complex [GO:0140513]; is part of GO:0005654; BFO_0000051 origin recognition complex [GO:0000808]; has part MCM complex [GO:0042555]